{
  "gene_symbol": "CYP2U1",
  "term_label": "heme binding",
  "gene_name": "Cytochrome P450 2U1",
  "gene": "UniProtKB:Q7Z449",
  "term_id": "GO:0020037"
}